{
  "gene": "UniProtKB:Q03113",
  "term_label": "heterotrimeric G-protein complex",
  "gene_name": "Guanine nucleotide-binding protein subunit alpha-12",
  "gene_symbol": "GNA12",
  "term_id": "GO:0005834"
}